{
  "term_label": "Unknown biological process",
  "gene_name": "Tyrosine-protein kinase ZAP-70",
  "gene_symbol": "ZAP70",
  "term_id": "UNKNOWN:0002",
  "gene": "UniProtKB:P43403"
}